(-)-exo-alpha-bergamotene catabolic process [GO:1901939] (biological process) References: PMID:22867794 Sources: GOC:TermGenie Also known as: (-)-exo-alpha-bergamotene breakdown, (-)-exo-alpha-bergamotene catabolism, (-)-exo-alpha-bergamotene degradation Definition: The chemical reactions and pathways resulting in the breakdown of (-)-exo-alpha-bergamotene. Relationships: is_a sesquiterpene catabolic process [GO:0051763]; is a type of olefinic compound catabolic process [GO:0120256]; is_a olefin metabolic process [GO:1900673]